symbiont-mediated transformation of host cell [GO:0019087] (biological process) Definition: A symbiont-induced cellular transformation resulting in immortalized cells, or cells capable of indefinite replication. Usually mediated by viruses. References: PMID:11119620, PMID:18366075, PMID:24373315 Sources: ISBN:0781702534 Also known as: host cell immortalization, host cell transformation, immortalization of host cell, transformation of host cell, transformation of host cell by virus, viral immortalization, viral transformation, viral transformation of host cell, immortalization of host cell by virus, virus-mediated transformation of host cell Relationships: is a type of symbiont-mediated perturbation of host cellular process [GO:0044068] Regulation: regulated by regulation of transformation of host cell by virus [GO:1904187]; negatively regulated by negative regulation of transformation of host cell by virus [GO:1904188]; positively regulated by positive regulation of transformation of host cell by virus [GO:1904189]